{
  "term_label": "leukemia inhibitory factor signaling pathway",
  "term_id": "GO:0048861",
  "gene_name": "Leukemia inhibitory factor",
  "gene_symbol": "LIF",
  "gene": "UniProtKB:P15018"
}